{
  "gene_symbol": "RAD23A",
  "gene_name": "UV excision repair protein RAD23 homolog A",
  "term_id": "GO:0031593",
  "gene": "UniProtKB:P54725",
  "term_label": "polyubiquitin modification-dependent protein binding"
}